{
  "term_id": "UNKNOWN:0001",
  "gene": "UniProtKB:A0A0C4DH24",
  "gene_name": "Immunoglobulin kappa variable 6-21",
  "gene_symbol": "IGKV6-21",
  "term_label": "Unknown molecular function"
}